{
  "term_id": "GO:0005634",
  "term_label": "nucleus",
  "gene_name": "Probable ribonuclease ZC3H12B",
  "gene_symbol": "ZC3H12B",
  "gene": "UniProtKB:Q5HYM0"
}